{
  "term_label": "regulation of cardiac muscle contraction by regulation of the release of sequestered calcium ion",
  "gene_symbol": "FKBP1B",
  "gene": "UniProtKB:P68106",
  "gene_name": "Peptidyl-prolyl cis-trans isomerase FKBP1B",
  "term_id": "GO:0010881"
}